glycerophosphodiester transmembrane transporter activity [GO:0001406] (molecular function) Definition: Enables the transfer of glycerophosphodiesters from one side of a membrane to the other. Glycerophosphodiesters are small molecules composed of glycerol-3-phosphate and an alcohol, for example, glycerophosphoinositol. References: PMID:12912892 Sources: GOC:mcc Relationships: is a type of GO:0015605; is part of glycerophosphodiester transmembrane transport [GO:0001407]